{
  "term_label": "mitochondrial RNA 3'-end processing",
  "term_id": "GO:0000965",
  "gene_symbol": "PNPT1",
  "gene_name": "Polyribonucleotide nucleotidyltransferase 1, mitochondrial",
  "gene": "UniProtKB:Q8TCS8"
}